{
  "gene_name": "DnaJ homolog subfamily B member 5",
  "gene_symbol": "DNAJB5",
  "term_id": "GO:0006457",
  "gene": "UniProtKB:O75953",
  "term_label": "protein folding"
}